{
  "term_label": "cytoplasm",
  "gene_name": "Secreted frizzled-related protein 4",
  "gene_symbol": "SFRP4",
  "gene": "UniProtKB:Q6FHJ7",
  "term_id": "GO:0005737"
}